{
  "term_id": "GO:0034702",
  "gene": "UniProtKB:Q7L1W4",
  "gene_symbol": "LRRC8D",
  "gene_name": "Volume-regulated anion channel subunit LRRC8D",
  "term_label": "monoatomic ion channel complex"
}